{
  "gene_name": "Potassium_sodium hyperpolarization-activated cyclic nucleotide-gated channel 3",
  "term_id": "GO:0071805",
  "term_label": "potassium ion transmembrane transport",
  "gene": "UniProtKB:Q9P1Z3",
  "gene_symbol": "HCN3"
}